{
  "gene": "UniProtKB:A0N4X5",
  "term_id": "UNKNOWN:0003",
  "gene_name": "HCG2039756 (Fragment)",
  "gene_symbol": "TRAJ34",
  "term_label": "Unknown cellular component"
}